split septin rings [GO:0032176] (cellular component) Subtypes: GO:0032177 References: PMID:16009555, PMID:16151244 Sources: GOC:krc Relationships: is a type of septin cytoskeleton [GO:0032156]; is part of cytoskeleton [GO:0005856] Definition: A pair of rings that flank the site of cell division, formed by splitting of the septin ring (or collar) prior to cytokinesis; this double ring structure is thought to trap proteins needed for cytokinesis or the formation of the new membrane or cell wall between the two septin rings. Split septin rings are known to occur in budding yeast cells and probably occur in other cell types as well.